{
  "gene_symbol": "TOM1",
  "gene_name": "Target of Myb1 membrane trafficking protein",
  "term_label": "membrane",
  "gene": "UniProtKB:O60784",
  "term_id": "GO:0016020"
}